arginine N-succinyltransferase activity [GO:0008791] (molecular function) Also known as: AOST activity, AST activity, AstA, arginine and ornithine N(2)-succinyltransferase activity, arginine and ornithine N2-succinyltransferase activity, arginine succinyltransferase activity, succinyl-CoA:L-arginine 2-N-succinyltransferase activity, succinyl-CoA:L-arginine N2-succinyltransferase activity Sources: EC:2.3.1.109 Definition: Catalysis of the reaction: succinyl-CoA + L-arginine = CoA + N2-succinyl-L-arginine. Relationships: is a type of GO:0016749